{
  "term_id": "GO:0032040",
  "term_label": "small-subunit processome",
  "gene": "UniProtKB:Q9NQZ2",
  "gene_symbol": "UTP3",
  "gene_name": "Something about silencing protein 10"
}